negative regulation of immune response to tumor cell [GO:0002838] (biological process) Sources: GOC:add Also known as: down regulation of immune response to tumor cell, down-regulation of immune response to tumor cell, downregulation of immune response to tumor cell, negative regulation of immune response to tumour cell, inhibition of immune response to tumor cell Subtypes: GO:0002841, negative regulation of tolerance induction to tumor cell [GO:0002844], negative regulation of natural killer cell mediated immune response to tumor cell [GO:0002856] Relationships: is_a negative regulation of response to tumor cell [GO:0002835]; is_a regulation of immune response to tumor cell [GO:0002837]; is_a negative regulation of immune response [GO:0050777]; negatively regulates immune response to tumor cell [GO:0002418] Definition: Any process that stops, prevents, or reduces the frequency, rate, or extent of an immune response to tumor cell.